{
  "gene": "UniProtKB:Q9H1B4",
  "term_id": "GO:0005634",
  "term_label": "nucleus",
  "gene_symbol": "NXF5",
  "gene_name": "Nuclear RNA export factor 5"
}